{
  "gene_symbol": "STOX2",
  "gene_name": "Storkhead-box protein 2",
  "term_label": "nucleus",
  "gene": "UniProtKB:Q9P2F5",
  "term_id": "GO:0005634"
}